negative regulation of germ cell proliferation [GO:1905937] (biological process) Relationships: is a type of negative regulation of cell population proliferation [GO:0008285]; is_a GO:0051241; is_a regulation of germ cell proliferation [GO:1905936]; negatively regulates germ cell proliferation [GO:0036093] Definition: Any process that stops, prevents or reduces the frequency, rate or extent of germ cell proliferation. Subtypes: GO:2000255 Also known as: down regulation of germ cell proliferation, down-regulation of germ cell proliferation, downregulation of germ cell proliferation, inhibition of germ cell proliferation References: PMID:15342467 Sources: GOC:TermGenie, GO_REF:0000058